root development [GO:0048364] (biological process) Definition: The process whose specific outcome is the progression of the root over time, from its formation to the mature structure. The root is the water- and mineral-absorbing part of a plant which is usually underground, does not bear leaves, tends to grow downwards and is typically derived from the radicle of the embryo. Relationships: is a type of plant organ development [GO:0099402]; is part of GO:0022622 Subtypes: post-embryonic root development [GO:0048528], GO:0048830, GO:0062211, primary root development [GO:0080022] Sources: GOC:jid, PO:0009005 Regulation: regulated by regulation of root development [GO:2000280]